{
  "gene_symbol": "RGSL1",
  "gene": "UniProtKB:A5PLK6",
  "gene_name": "Regulator of G-protein signaling protein-like",
  "term_label": "Unknown biological process",
  "term_id": "UNKNOWN:0002"
}